{
  "term_id": "GO:0003735",
  "gene": "UniProtKB:P61247",
  "gene_symbol": "RPS3A",
  "gene_name": "Small ribosomal subunit protein eS1",
  "term_label": "structural constituent of ribosome"
}